{
  "term_id": "GO:0004672",
  "gene": "UniProtKB:P00540",
  "gene_name": "Proto-oncogene serine_threonine-protein kinase mos",
  "term_label": "protein kinase activity",
  "gene_symbol": "MOS"
}